{
  "term_label": "protein localization to plasma membrane",
  "gene": "UniProtKB:Q8IXS8",
  "term_id": "GO:0072659",
  "gene_name": "Hyccin 2",
  "gene_symbol": "HYCC2"
}